negative regulation of lncRNA transcription [GO:0140744] (biological process) Relationships: is_a negative regulation of DNA-templated transcription [GO:0045892]; is a type of regulation of lncRNA transcription [GO:0140743]; negatively regulates lncRNA transcription [GO:0140742] References: PMID:33767452, PMID:33913806 Definition: Any process that decreases the frequency, rate or extent of the synthesis of a lncRNA.